host cell outer membrane [GO:0039662] (cellular component) Relationships: is a type of host outer membrane [GO:0044384]; is part of host cell envelope [GO:0044230] Definition: A lipid bilayer that forms the outermost layer of the cell envelope, occurring in a host cell. Also known as: host cell envelope outer membrane, outer membrane of host cell Sources: GOC:bf, GOC:ch